{
  "term_label": "proton-transporting ATP synthase activity, rotational mechanism",
  "term_id": "GO:0046933",
  "gene_symbol": "ATP5MG",
  "gene": "UniProtKB:O75964",
  "gene_name": "ATP synthase subunit g, mitochondrial"
}